{
  "term_label": "Unknown molecular function",
  "gene_symbol": "TRAJ53",
  "gene": "UniProtKB:A0A075B6W9",
  "term_id": "UNKNOWN:0001",
  "gene_name": "T cell receptor alpha joining 53 (Fragment)"
}